positive regulation of membrane repolarization during cardiac muscle cell action potential [GO:1905033] (biological process) Definition: Any process that activates or increases the frequency, rate or extent of membrane repolarization during cardiac muscle cell action potential. References: PMID:23157812 Sources: GOC:BHF, GOC:BHF_miRNA, GOC:TermGenie, GOC:mtg_cardiac_conduct_nov11, GOC:rph Also known as: up regulation of membrane repolarization during cardiac muscle cell action potential, up-regulation of membrane repolarization during cardiac muscle cell action potential, upregulation of membrane repolarization during cardiac muscle cell action potential, activation of membrane repolarization during cardiac muscle cell action potential Relationships: is a type of positive regulation of biological process [GO:0048518]; is a type of regulation of membrane repolarization during cardiac muscle cell action potential [GO:1905031]; positively regulates membrane repolarization during cardiac muscle cell action potential [GO:0086013] Subtypes: GO:1905002, positive regulation of membrane repolarization during ventricular cardiac muscle cell action potential [GO:1905026]